{
  "gene": "UniProtKB:Q9NQC1",
  "gene_name": "E3 ubiquitin-protein ligase Jade-2",
  "term_id": "GO:0006338",
  "gene_symbol": "JADE2",
  "term_label": "chromatin remodeling"
}